cell-cell junction [GO:0005911] (CC) Also known as: cell-cell contact region, cell-cell contact zone, intercellular junction Subtypes: adherens junction [GO:0005912], fascia adherens [GO:0005916], gap junction [GO:0005921], plasmodesma [GO:0009506], desmosome [GO:0030057], paranodal junction [GO:0033010], filtration diaphragm [GO:0036056], apical junction complex [GO:0043296], cell-cell contact zone [GO:0044291], GO:0046581, apical ectoplasmic specialization [GO:0061831], basal ectoplasmic specialization [GO:0061832], tight junction [GO:0070160] Relationships: is a type of anchoring junction [GO:0070161] References: PMID:21422226, PMID:28096264 Sources: GOC:aruk, GOC:bc, GOC:dgh, GOC:hb, GOC:mah Definition: A cell junction that forms a connection between two or more cells of an organism; excludes direct cytoplasmic intercellular bridges, such as ring canals in insects.